{
  "gene_symbol": "HNRNPD",
  "term_label": "nucleoplasm",
  "gene_name": "Heterogeneous nuclear ribonucleoprotein D0",
  "gene": "UniProtKB:Q14103",
  "term_id": "GO:0005654"
}